{
  "gene_name": "Ubiquinone biosynthesis monooxygenase COQ6, mitochondrial",
  "term_id": "GO:0016491",
  "gene_symbol": "COQ6",
  "gene": "UniProtKB:Q9Y2Z9",
  "term_label": "oxidoreductase activity"
}